{
  "gene": "UniProtKB:Q9BVI4",
  "gene_symbol": "NOC4L",
  "gene_name": "Nucleolar complex protein 4 homolog",
  "term_id": "UNKNOWN:0002",
  "term_label": "Unknown biological process"
}